{
  "term_id": "UNKNOWN:0001",
  "gene_name": "Tetratricopeptide repeat protein 12",
  "gene": "UniProtKB:Q9H892",
  "gene_symbol": "TTC12",
  "term_label": "Unknown molecular function"
}